{
  "gene": "UniProtKB:P41214",
  "gene_name": "Eukaryotic translation initiation factor 2D",
  "term_label": "Unknown cellular component",
  "gene_symbol": "EIF2D",
  "term_id": "UNKNOWN:0003"
}